{
  "gene_name": "Small RNA 2'-O-methyltransferase",
  "term_label": "RNA methyltransferase activity",
  "gene": "UniProtKB:Q5T8I9",
  "gene_symbol": "HENMT1",
  "term_id": "GO:0008173"
}